{
  "gene_symbol": "BAGE",
  "gene": "UniProtKB:Q13072",
  "gene_name": "B melanoma antigen 1",
  "term_id": "UNKNOWN:0002",
  "term_label": "Unknown biological process"
}